histoblast morphogenesis [GO:0007488] (biological process) Also known as: histoblast metamorphosis Definition: The process in which the anatomical structures derived from the histoblast disc are generated and organized. This includes the transformation of histoblast cells into adult structures during pupal metamorphosis. Histoblast cells are cells founded in the embryo that are the progenitors to the adult abdomen. Sources: GOC:bf, ISBN:0879694238 Relationships: is a type of cell morphogenesis [GO:0000902]; is a type of imaginal disc morphogenesis [GO:0007560]